{
  "gene_name": "Cryptochrome-1",
  "gene": "UniProtKB:Q16526",
  "term_label": "entrainment of circadian clock by photoperiod",
  "gene_symbol": "CRY1",
  "term_id": "GO:0043153"
}